{
  "gene_name": "Receptor tyrosine-protein kinase erbB-2",
  "gene": "UniProtKB:P04626",
  "term_label": "receptor complex",
  "term_id": "GO:0043235",
  "gene_symbol": "ERBB2"
}